{
  "gene_name": "Kunitz-type protease inhibitor 4",
  "gene_symbol": "SPINT4",
  "term_id": "UNKNOWN:0003",
  "gene": "UniProtKB:Q6UDR6",
  "term_label": "Unknown cellular component"
}